sweat secretion [GO:0160269] (biological process) Definition: The regulated release of sweat from the sweat glands. References: PMID:1778649 Also known as: perspiration, perspiring, sweating Relationships: is a type of body fluid secretion [GO:0007589]; is a type of secretion by tissue [GO:0032941]